eukaryotic translation initiation factor 4F complex assembly [GO:0097010] (biological process) Regulation: regulated by regulation of eukaryotic translation initiation factor 4F complex assembly [GO:1905535]; negatively regulated by negative regulation of eukaryotic translation initiation factor 4F complex assembly [GO:1905536]; positively regulated by positive regulation of eukaryotic translation initiation factor 4F complex assembly [GO:1905537] References: PMID:18337562 Sources: GOC:BHF, GOC:ebc Also known as: eIF-4F assembly, eIF4F assembly Definition: The aggregation, arrangement and bonding together of a set of components to form the eukaryotic translation initiation factor 4F complex. Relationships: is a type of protein-containing complex assembly [GO:0065003]